regulation of acrosome reaction [GO:0060046] (biological process) Relationships: is a type of regulation of reproductive process [GO:2000241]; regulates acrosome reaction [GO:0007340] Definition: Any process that modulates the frequency, rate or extent of the acrosome reaction. Sources: GOC:dph Subtypes: negative regulation of acrosome reaction [GO:1902225], positive regulation of acrosome reaction [GO:2000344]